{
  "gene": "UniProtKB:Q2L4Q9",
  "term_id": "UNKNOWN:0002",
  "gene_name": "Serine protease 53",
  "gene_symbol": "PRSS53",
  "term_label": "Unknown biological process"
}